pheromone-induced unidirectional conjugation [GO:0000762] (biological process) Regulation: regulated by response to pheromone regulating pheromone-induced unidirectional conjugation [GO:0000765] Definition: Unidirectional transfer of genetic information triggered by to a pheromone signal. References: PMID:17360276, PMID:27021562, PMID:31191478 Sources: GOC:elh Relationships: is a type of unidirectional conjugation [GO:0009291]